{
  "gene": "UniProtKB:Q12756",
  "term_label": "microtubule binding",
  "gene_symbol": "KIF1A",
  "term_id": "GO:0008017",
  "gene_name": "Kinesin-like protein KIF1A"
}